{
  "gene_symbol": "CREBL2",
  "gene_name": "cAMP-responsive element-binding protein-like 2",
  "gene": "UniProtKB:O60519",
  "term_id": "GO:0005634",
  "term_label": "nucleus"
}